{
  "gene": "UniProtKB:O60573",
  "term_label": "translational initiation",
  "gene_symbol": "EIF4E2",
  "gene_name": "Eukaryotic translation initiation factor 4E type 2",
  "term_id": "GO:0006413"
}